regulation of myeloid progenitor cell differentiation [GO:1905453] (biological process) Definition: Any process that modulates the frequency, rate or extent of myeloid progenitor cell differentiation. References: PMID:27010503 Sources: GOC:TermGenie, GO_REF:0000058 Relationships: is a type of regulation of hematopoietic progenitor cell differentiation [GO:1901532]; regulates GO:0002318 Subtypes: negative regulation of myeloid progenitor cell differentiation [GO:1905454], positive regulation of myeloid progenitor cell differentiation [GO:1905455]